{
  "gene": "UniProtKB:Q8IYX3",
  "term_label": "Unknown molecular function",
  "gene_name": "Coiled-coil domain-containing protein 116",
  "gene_symbol": "CCDC116",
  "term_id": "UNKNOWN:0001"
}